{
  "gene": "UniProtKB:Q969T7",
  "term_id": "UNKNOWN:0002",
  "gene_symbol": "NT5C3B",
  "gene_name": "7-methylguanosine phosphate-specific 5'-nucleotidase",
  "term_label": "Unknown biological process"
}